{
  "gene_symbol": "ZNF92",
  "term_label": "Unknown cellular component",
  "gene": "UniProtKB:Q03936",
  "term_id": "UNKNOWN:0003",
  "gene_name": "Zinc finger protein 92"
}